neuropeptide signaling pathway [GO:0007218] (biological process) Sources: GOC:mah, ISBN:0815316194 Subtypes: galanin-activated signaling pathway [GO:0090663] Definition: A G protein-coupled receptor signaling pathway initiated by a neuropeptide binding to its receptor on the surface of a target cell, and ending with the regulation of a downstream cellular process. Also known as: neuropeptide signalling pathway Relationships: is a type of G protein-coupled receptor signaling pathway [GO:0007186]